{
  "gene_symbol": "KCND2",
  "gene_name": "Potassium voltage-gated channel subfamily D member 2",
  "gene": "UniProtKB:Q9NZV8",
  "term_id": "GO:0043025",
  "term_label": "neuronal cell body"
}